{
  "gene_symbol": "CLDN7",
  "gene": "UniProtKB:O95471",
  "gene_name": "Claudin-7",
  "term_label": "cell-cell junction organization",
  "term_id": "GO:0045216"
}